galactarate transmembrane transport [GO:1902300] (biological process) Sources: GOC:TermGenie, GOC:pr Relationships: is a type of aldarate transmembrane transport [GO:0042869] Definition: The process in which galactaric acid anion (galactarate) is transported across a lipid bilayer, from one side of a membrane to the other. Also known as: galactaric acid anion transport, D-galactarate transport, galactarate transport